stimulatory C-type lectin receptor signaling pathway [GO:0002223] (BP) Definition: The series of molecular signals initiated by the binding of C-type lectin to its receptor on the surface of a target cell, and resulting in cellular activation. Sources: GOC:add, GO_REF:0000022, ISBN:0781735149 Also known as: stimulatory C-type lectin receptor signalling pathway, stimulatory Ly49 family receptor signaling pathway Relationships: is a type of innate immune response activating cell surface receptor signaling pathway [GO:0002220]; is a type of cellular response to lectin [GO:1990858]